{
  "gene_name": "DNA polymerase delta catalytic subunit",
  "gene_symbol": "POLD1",
  "term_label": "DNA replication proofreading",
  "gene": "UniProtKB:P28340",
  "term_id": "GO:0045004"
}